{
  "gene_name": "Fanconi anemia group M protein",
  "gene_symbol": "FANCM",
  "gene": "UniProtKB:Q8IYD8",
  "term_id": "UNKNOWN:0003",
  "term_label": "Unknown cellular component"
}